{
  "term_label": "manganese ion binding",
  "term_id": "GO:0030145",
  "gene": "UniProtKB:Q3LIE5",
  "gene_symbol": "ADPRM",
  "gene_name": "Manganese-dependent ADP-ribose_CDP-alcohol diphosphatase"
}